{
  "gene": "UniProtKB:Q9BS40",
  "term_label": "extracellular space",
  "gene_symbol": "LXN",
  "gene_name": "Latexin",
  "term_id": "GO:0005615"
}